{
  "gene_symbol": "STMN3",
  "gene": "UniProtKB:Q9NZ72",
  "term_label": "regulation of microtubule polymerization or depolymerization",
  "gene_name": "Stathmin-3",
  "term_id": "GO:0031110"
}